{
  "gene_symbol": "LIMD1",
  "term_id": "GO:0005634",
  "term_label": "nucleus",
  "gene_name": "LIM domain-containing protein 1",
  "gene": "UniProtKB:Q9UGP4"
}